UTP-monosaccharide-1-phosphate uridylyltransferase activity [GO:0051748] (molecular function) Definition: Catalysis of the reaction: UTP + a monosaccharide 1-phosphate = diphosphate + UDP-monosaccharide. References: PMID:15326166 Sources: EC:2.7.7.64 Subtypes: GO:0003983, UTP:arabinose-1-phosphate uridylyltransferase activity [GO:0010491], UTP:galactose-1-phosphate uridylyltransferase activity [GO:0017103], GO:0047338 Also known as: UDP-monosaccharide diphosphorylase activity, UDP-monosaccharide pyrophosphorylase activity, PsUSP, UDP-sugar pyrophosphorylase activity, USP Relationships: is a type of uridylyltransferase activity [GO:0070569]